5-methyltetrahydrofolate-dependent methyltransferase activity [GO:0042084] (molecular function) Subtypes: methionine synthase activity [GO:0008705] Sources: GOC:ai Definition: Catalysis of the transfer of a methyl group to an acceptor molecule; dependent on the presence of 5-methyltetrahydrofolate. Relationships: is a type of methyltransferase activity [GO:0008168]